{
  "gene_name": "Interleukin-1 beta",
  "gene_symbol": "IL1B",
  "gene": "UniProtKB:P01584",
  "term_id": "GO:0005615",
  "term_label": "extracellular space"
}